{
  "term_id": "GO:0004741",
  "term_label": "[pyruvate dehydrogenase (acetyl-transferring)]-phosphatase activity",
  "gene_symbol": "PDP1",
  "gene_name": "[Pyruvate dehydrogenase [acetyl-transferring]]-phosphatase 1, mitochondrial",
  "gene": "UniProtKB:Q9P0J1"
}